{
  "gene_symbol": "EIF2B4",
  "gene_name": "Translation initiation factor eIF-2B subunit delta",
  "term_label": "Unknown molecular function",
  "gene": "UniProtKB:Q9UI10",
  "term_id": "UNKNOWN:0001"
}